{
  "term_id": "GO:0061024",
  "term_label": "membrane organization",
  "gene": "UniProtKB:Q99961",
  "gene_symbol": "SH3GL1",
  "gene_name": "Endophilin-A2"
}